effector-mediated perturbation of host innate immune response by symbiont [GO:0140404] (BP) Relationships: is a type of symbiont-mediated perturbation of host innate immune response [GO:0052167]; is a type of effector-mediated perturbation of host defenses by symbiont [GO:0140415] Subtypes: effector-mediated suppression of host innate immune response [GO:0140403], effector-mediated suppression of host salicylic acid-mediated innate immune signaling [GO:0140502] Also known as: effector mediated modulation of host immune response by symbiont, effector triggered modulation of host immune response by symbiont, effector-dependent modulation of host immune response by symbiont, effector-mediated modulation of host immunity, effector-mediated modulation of host innate immune response by symbiont, effector-triggered modulation of host immune response by symbiont Definition: A process mediated by a molecule secreted by a symbiont that results in the modulation (either activation or suppression) of a host innate immune response. The host is defined as the larger of the organisms involved in a symbiotic interaction. References: PMID:21467214